{
  "term_id": "GO:0016477",
  "gene_symbol": "NDE1",
  "gene": "UniProtKB:Q9NXR1",
  "gene_name": "Nuclear distribution protein nudE homolog 1",
  "term_label": "cell migration"
}